{
  "gene": "UniProtKB:I0J062",
  "gene_symbol": "PANO1",
  "term_id": "UNKNOWN:0002",
  "term_label": "Unknown biological process",
  "gene_name": "Proapoptotic nucleolar protein 1"
}